deoxyuridine metabolic process [GO:0046096] (biological process) Subtypes: GO:0006219, GO:0046097 Definition: The chemical reactions and pathways involving deoxyuridine, 2-deoxyribosyluracil, one of the four major nucleosides of DNA. Sources: GOC:go_curators Relationships: is a type of GO:0046125 Also known as: deoxyuridine metabolism